{
  "term_label": "signaling receptor binding",
  "gene_symbol": "THPO",
  "term_id": "GO:0005102",
  "gene": "UniProtKB:P40225",
  "gene_name": "Thrombopoietin"
}